{
  "term_id": "GO:0061630",
  "gene_name": "E3 ubiquitin-protein ligase RNF5",
  "term_label": "ubiquitin protein ligase activity",
  "gene_symbol": "RNF5",
  "gene": "UniProtKB:Q99942"
}